{
  "gene_name": "Zinc finger protein 443",
  "gene_symbol": "ZNF443",
  "term_id": "GO:0005634",
  "gene": "UniProtKB:Q9Y2A4",
  "term_label": "nucleus"
}